{
  "gene_symbol": "MYH13",
  "term_label": "myosin filament",
  "term_id": "GO:0032982",
  "gene_name": "Myosin-13",
  "gene": "UniProtKB:Q9UKX3"
}